{
  "gene": "UniProtKB:Q92552",
  "term_label": "Unknown biological process",
  "term_id": "UNKNOWN:0002",
  "gene_name": "Small ribosomal subunit protein mS27",
  "gene_symbol": "MRPS27"
}